{
  "gene_name": "B-cell CLL_lymphoma 7 protein family member A",
  "term_label": "Unknown cellular component",
  "gene_symbol": "BCL7A",
  "gene": "UniProtKB:Q4VC05",
  "term_id": "UNKNOWN:0003"
}